{
  "gene_name": "Potassium channel subfamily K member 17",
  "term_label": "potassium ion leak channel activity",
  "term_id": "GO:0022841",
  "gene": "UniProtKB:Q96T54",
  "gene_symbol": "KCNK17"
}